{
  "gene": "UniProtKB:P31941",
  "term_id": "GO:0045869",
  "gene_symbol": "APOBEC3A",
  "gene_name": "DNA dC-dU-editing enzyme APOBEC-3A",
  "term_label": "negative regulation of single stranded viral RNA replication via double stranded DNA intermediate"
}